{
  "gene_symbol": "RUNX3",
  "term_label": "chondrocyte differentiation",
  "gene_name": "Runt-related transcription factor 3",
  "gene": "UniProtKB:Q13761",
  "term_id": "GO:0002062"
}